{
  "gene_symbol": "RIOK1",
  "gene": "UniProtKB:Q9BRS2",
  "term_label": "maturation of SSU-rRNA",
  "gene_name": "Serine_threonine-protein kinase RIO1",
  "term_id": "GO:0030490"
}